glutamate receptor activity [GO:0008066] (molecular function) Definition: Combining with glutamate and transmitting the signal from one side of the membrane to the other to initiate a change in cell activity. Relationships: is a type of transmembrane signaling receptor activity [GO:0004888]; BFO_0000051 GO:0016595 Sources: GOC:ai, GOC:signaling Subtypes: glutamate-gated receptor activity [GO:0004970], GO:0098988